{
  "gene_symbol": "FEZ1",
  "term_label": "cytoplasm",
  "term_id": "GO:0005737",
  "gene_name": "Fasciculation and elongation protein zeta-1",
  "gene": "UniProtKB:Q99689"
}